ubiquitin-like protein ligase activity [GO:0061659] (molecular function) Subtypes: Atg8-family ligase activity [GO:0019776], ubiquitin protein ligase activity [GO:0061630], Atg12 ligase activity [GO:0061660], GO:0061661, ISG15 ligase activity [GO:0061662], NEDD8 ligase activity [GO:0061663], GO:0061664, SUMO ligase activity [GO:0061665], UFM1 ligase activity [GO:0061666], GO:0061667 Sources: GOC:dph Also known as: small conjugating protein ligase activity, E3 Relationships: is a type of ubiquitin-like protein transferase activity [GO:0019787] Definition: Catalysis of the transfer of a ubiquitin-like protein (ULP) to a substrate protein via the reaction X-ULP + S = X + S-ULP, where X is either an E2 or E3 enzyme, the X-ULP linkage is a thioester bond, and the S-ULP linkage is an isopeptide bond between the C-terminal glycine of ULP and the epsilon-amino group of lysine residues in the substrate.